{
  "term_id": "GO:0030337",
  "gene_name": "Proliferating cell nuclear antigen",
  "gene": "UniProtKB:P12004",
  "term_label": "DNA polymerase processivity factor activity",
  "gene_symbol": "PCNA"
}